{
  "term_id": "GO:0035861",
  "term_label": "site of double-strand break",
  "gene_symbol": "PARP3",
  "gene_name": "Protein mono-ADP-ribosyltransferase PARP3",
  "gene": "UniProtKB:Q9Y6F1"
}